{
  "gene_symbol": "CSF2RA",
  "term_label": "cytokine binding",
  "gene_name": "Granulocyte-macrophage colony-stimulating factor receptor subunit alpha",
  "term_id": "GO:0019955",
  "gene": "UniProtKB:P15509"
}